{
  "gene_name": "Rieske domain-containing protein",
  "gene": "UniProtKB:Q8TAC1",
  "gene_symbol": "RFESD",
  "term_id": "UNKNOWN:0002",
  "term_label": "Unknown biological process"
}